pectate lyase activity [GO:0030570] (molecular function) Also known as: pectic lyase activity, pectin trans-eliminase activity, (1->4)-alpha-D-galacturonan lyase activity, PGA lyase activity, PPase-N activity, alpha-1,4-D-endopolygalacturonic acid lyase activity, endo-alpha-1,4-polygalacturonic acid lyase activity, endogalacturonate transeliminase activity, endopectin methyltranseliminase activity, pectate transeliminase activity, pectic acid lyase activity, pectic acid transeliminase activity, polygalacturonate lyase activity, polygalacturonic acid lyase activity, polygalacturonic acid trans-eliminase activity, polygalacturonic transeliminase activity Definition: Catalysis of the reaction: a pectate = a pectate + a pectate oligosaccharide with 4-(4-deoxy-alpha-D-galact-4-enuronosyl)-D-galacturonate end. This reaction is the eliminative cleavage of pectate to give oligosaccharides with 4-deoxy-alpha-D-gluc-4-enuronosyl groups at their non-reducing ends. Sources: EC:4.2.2.2 Relationships: is a type of carbon-oxygen lyase activity, acting on polysaccharides [GO:0016837]